thymine catabolic process [GO:0006210] (BP) Also known as: thymine breakdown, thymine catabolism, thymine degradation Relationships: is_a pyrimidine nucleobase catabolic process [GO:0006208]; is a type of thymine metabolic process [GO:0019859] Definition: The chemical reactions and pathways resulting in the breakdown of thymine, 5-methyluracil, one of the two major pyrimidine bases present (as thymidine) in DNA but not found in RNA other than (as ribothymidine) in transfer RNA, where it is a minor base. Sources: GOC:go_curators